inositol monophosphate 4-phosphatase activity [GO:0052833] (molecular function) Definition: Catalysis of the reaction:1D-myo-inositol 4-phosphate + H2O = myo-inositol + phosphate. Relationships: is a type of inositol monophosphate phosphatase activity [GO:0052834] Sources: RHEA:30735 Also known as: inositol-1(or 4)-monophosphatase activity, myo-inositol-1(or 4)-monophosphatase activity, myo-inositol-1(or 4)-phosphate phosphohydrolase activity